{
  "gene": "UniProtKB:P51511",
  "gene_symbol": "MMP15",
  "term_label": "extracellular space",
  "gene_name": "Matrix metalloproteinase-15",
  "term_id": "GO:0005615"
}